{
  "term_label": "molecular adaptor activity",
  "gene_symbol": "DLGAP3",
  "term_id": "GO:0060090",
  "gene_name": "Disks large-associated protein 3",
  "gene": "UniProtKB:O95886"
}